regulation of DNA stability [GO:0097752] (biological process) Relationships: is_a regulation of biological quality [GO:0065008] Sources: GOC:pr Definition: Any process that modulates the stability of DNA.